{
  "gene_symbol": "TMEM69",
  "term_id": "UNKNOWN:0003",
  "term_label": "Unknown cellular component",
  "gene": "UniProtKB:Q5SWH9",
  "gene_name": "Transmembrane protein 69"
}